response to hypoxia [GO:0001666] (biological process) Note: Note that this term should not be confused with 'response to anoxia ; GO:0034059'. Note that in laboratory studies, hypoxia is typically studied at O2 concentrations ranging from 0.1 - 5%. Definition: Any process that results in a change in state or activity of a cell or an organism (in terms of movement, secretion, enzyme production, gene expression, etc.) as a result of a stimulus indicating lowered oxygen tension. Hypoxia, defined as a decline in O2 levels below normoxic levels of 20.8 - 20.95%, results in metabolic adaptation at both the cellular and organismal level. Relationships: is a type of response to stress [GO:0006950]; is a type of response to decreased oxygen levels [GO:0036293] Subtypes: detection of hypoxia [GO:0070483], cellular response to hypoxia [GO:0071456], response to hypobaric hypoxia [GO:1990910] Also known as: response to hypoxic stress, response to lowered oxygen tension, response to intermittent hypoxia, response to sustained hypoxia Sources: GOC:hjd